angiotensin-mediated vasoconstriction involved in regulation of systemic arterial blood pressure [GO:0001998] (biological process) Also known as: angiotensin mediated vasoconstriction during blood pressure regulation, angiotensin mediated vasoconstriction involved in regulation of systemic arterial blood pressure, angiotensin mediated vasoconstriction during blood pressure control, angiotensin mediated vasoconstriction during control of blood pressure Sources: GOC:mtg_cardio, GOC:pr, ISBN:0721643949 Definition: The decrease in blood vessel diameter as a result of the release of angiotensin into the blood stream. Relationships: is_a positive regulation of systemic arterial blood pressure [GO:0003084]; is a type of vasoconstriction [GO:0042310]; is part of maintenance of blood vessel diameter homeostasis by renin-angiotensin [GO:0002034]